{
  "gene_name": "Protein Aster-C",
  "gene_symbol": "GRAMD1C",
  "gene": "UniProtKB:Q8IYS0",
  "term_id": "GO:0032366",
  "term_label": "intracellular sterol transport"
}